{
  "term_label": "DNA-binding transcription factor activity, RNA polymerase II-specific",
  "gene": "UniProtKB:A0A0U1RQI7",
  "gene_symbol": "KLF18",
  "gene_name": "Kruppel-like factor 18",
  "term_id": "GO:0000981"
}